{
  "term_label": "oxoglutarate dehydrogenase (succinyl-transferring) activity",
  "term_id": "GO:0004591",
  "gene_symbol": "OGDH",
  "gene_name": "2-oxoglutarate dehydrogenase complex component E1",
  "gene": "UniProtKB:Q02218"
}